positive regulation of inhibitory G protein-coupled receptor phosphorylation [GO:1904325] (biological process) Definition: Any process that activates or increases the frequency, rate or extent of inhibitory G protein-coupled receptor phosphorylation. Also known as: positive regulation of inhibitory G-protein coupled receptor phosphorylation, up regulation of inhibitory G-protein coupled receptor phosphorylation, up-regulation of inhibitory G-protein coupled receptor phosphorylation, upregulation of inhibitory G-protein coupled receptor phosphorylation, activation of inhibitory G-protein coupled receptor phosphorylation Relationships: is a type of positive regulation of protein phosphorylation [GO:0001934]; is a type of regulation of inhibitory G protein-coupled receptor phosphorylation [GO:1904323]; positively regulates GO:0002030 References: PMID:15937517 Sources: GOC:TermGenie, GO_REF:0000058